{
  "gene": "UniProtKB:Q8TCT6",
  "gene_name": "Signal peptide peptidase-like 3",
  "term_id": "GO:0030660",
  "gene_symbol": "SPPL3",
  "term_label": "Golgi-associated vesicle membrane"
}